inhibitory synapse [GO:0060077] (cellular component) Relationships: is a type of synapse [GO:0045202] Subtypes: GO:0098521, symmetric, GABA-ergic, inhibitory synapse [GO:0098983] Sources: GOC:dph, GOC:ef Definition: A synapse in which an action potential in the presynaptic cell reduces the probability of an action potential occurring in the postsynaptic cell.